{
  "gene_symbol": "OR6B3",
  "term_id": "UNKNOWN:0002",
  "gene": "UniProtKB:Q8NGW1",
  "term_label": "Unknown biological process",
  "gene_name": "Olfactory receptor 6B3"
}